{
  "term_label": "bitter taste receptor activity",
  "term_id": "GO:0033038",
  "gene_name": "Taste receptor type 2 member 5",
  "gene": "UniProtKB:Q9NYW4",
  "gene_symbol": "TAS2R5"
}